{
  "term_label": "ERAD pathway",
  "gene": "UniProtKB:Q99942",
  "gene_name": "E3 ubiquitin-protein ligase RNF5",
  "gene_symbol": "RNF5",
  "term_id": "GO:0036503"
}